{
  "term_label": "type I interferon-mediated signaling pathway",
  "gene": "UniProtKB:P01567",
  "gene_name": "Interferon alpha-7",
  "gene_symbol": "IFNA7",
  "term_id": "GO:0060337"
}